cranial nerve formation [GO:0021603] (biological process) Relationships: is a type of anatomical structure formation involved in morphogenesis [GO:0048646]; BFO_0000050 cranial nerve morphogenesis [GO:0021602] Sources: GOC:cls, GOC:dgh, GOC:dph, GOC:jid, GO_REF:0000021 Subtypes: GO:0021599, accessory nerve formation [GO:0021608], GO:0021611, glossopharyngeal nerve formation [GO:0021616], hypoglossal nerve formation [GO:0021620], oculomotor nerve formation [GO:0021623], olfactory nerve formation [GO:0021628], optic nerve formation [GO:0021634], trigeminal nerve formation [GO:0021638], trochlear nerve formation [GO:0021642], GO:0021646, GO:0021650 Definition: The process that gives rise to the cranial nerves. This process pertains to the initial formation of a structure from unspecified parts. The cranial nerves are composed of twelve pairs of nerves that emanate from the nervous tissue of the hindbrain. These nerves are sensory, motor, or mixed in nature, and provide the motor and general sensory innervation of the head, neck and viscera. They mediate vision, hearing, olfaction and taste and carry the parasympathetic innervation of the autonomic ganglia that control visceral functions.